{
  "gene": "UniProtKB:Q9BTV5",
  "term_label": "microtubule",
  "gene_symbol": "FSD1",
  "gene_name": "Fibronectin type III and SPRY domain-containing protein 1",
  "term_id": "GO:0005874"
}